{
  "term_id": "UNKNOWN:0001",
  "gene_name": "Osteoclast-stimulating factor 1",
  "gene_symbol": "OSTF1",
  "gene": "UniProtKB:Q92882",
  "term_label": "Unknown molecular function"
}